{
  "gene_symbol": "LSG1",
  "gene": "UniProtKB:Q9H089",
  "gene_name": "Large subunit GTPase 1 homolog",
  "term_label": "cytosol",
  "term_id": "GO:0005829"
}